shade avoidance [GO:0009641] (biological process) Definition: Shade avoidance is a set of responses that plants display when they are subjected to the shade of another plant. It often includes elongation, altered flowering time, increased apical dominance and altered partitioning of resources. Plants are able to distinguish between the shade of an inanimate object (e.g. a rock) and the shade of another plant due to the altered balance between red and far-red light in the shade of a plant; this balance between red and far-red light is perceived by phytochrome. Regulation: regulated by GO:1902446; negatively regulated by negative regulation of shade avoidance [GO:1902447]; positively regulated by positive regulation of shade avoidance [GO:1902448] Sources: Wikipedia:Shade_avoidance Relationships: is a type of response to red or far red light [GO:0009639]